{
  "gene_symbol": "ENPP4",
  "term_id": "UNKNOWN:0002",
  "gene": "UniProtKB:Q9Y6X5",
  "term_label": "Unknown biological process",
  "gene_name": "Bis(5'-adenosyl)-triphosphatase ENPP4"
}